{
  "term_id": "GO:0070936",
  "gene_symbol": "AMFR",
  "term_label": "protein K48-linked ubiquitination",
  "gene_name": "E3 ubiquitin-protein ligase AMFR",
  "gene": "UniProtKB:Q9UKV5"
}